{
  "gene_symbol": "PEPD",
  "gene_name": "Xaa-Pro dipeptidase",
  "term_label": "peptidase activity",
  "term_id": "GO:0008233",
  "gene": "UniProtKB:P12955"
}